rhombomere 8 morphogenesis [GO:0021674] (biological process) Definition: The process in which the anatomical structure of rhombomere 8 is generated and organized. Rhombomeres are transverse segments of the developing rhombencephalon. Rhombomeres are lineage restricted, express different genes from one another, and adopt different developmental fates. Rhombomeres are numbered in an anterior to posterior order. Relationships: is a type of rhombomere morphogenesis [GO:0021593]; is part of rhombomere 8 development [GO:0021574] Sources: GOC:cls, GOC:curators, GOC:dgh, GOC:dph, GOC:jid